{
  "term_id": "GO:0030007",
  "gene_symbol": "ATP1A2",
  "gene": "UniProtKB:P50993",
  "term_label": "intracellular potassium ion homeostasis",
  "gene_name": "Sodium_potassium-transporting ATPase subunit alpha-2"
}